{
  "term_label": "Unknown biological process",
  "gene_symbol": "ANKRD26P1",
  "gene_name": "Putative ankyrin repeat domain-containing protein 26-like protein",
  "term_id": "UNKNOWN:0002",
  "gene": "UniProtKB:Q6NSI1"
}